{
  "term_label": "C21-steroid hormone metabolic process",
  "gene": "UniProtKB:P14060",
  "term_id": "GO:0008207",
  "gene_symbol": "HSD3B1",
  "gene_name": "3 beta-hydroxysteroid dehydrogenase_Delta 5--4-isomerase type 1"
}